{
  "term_id": "GO:0000978",
  "gene": "UniProtKB:Q96CX3",
  "gene_symbol": "ZNF501",
  "term_label": "RNA polymerase II cis-regulatory region sequence-specific DNA binding",
  "gene_name": "Zinc finger protein 501"
}